negative regulation of saliva secretion [GO:1905747] (BP) Relationships: is a type of GO:0046877; is a type of negative regulation of secretion [GO:0051048]; is a type of negative regulation of digestive system process [GO:0060457]; negatively regulates saliva secretion [GO:0046541] Also known as: down regulation of saliva secretion, down regulation of salivation, down-regulation of saliva secretion, down-regulation of salivation, downregulation of saliva secretion, downregulation of salivation, negative regulation of salivation, inhibition of saliva secretion, inhibition of salivation References: PMID:23419067 Sources: GOC:TermGenie, GO_REF:0000058 Definition: Any process that stops, prevents or reduces the frequency, rate or extent of saliva secretion.